{
  "term_id": "GO:0042574",
  "gene": "UniProtKB:Q6PKH6",
  "gene_symbol": "DHRS4L2",
  "gene_name": "Dehydrogenase_reductase SDR family member 4-like 2",
  "term_label": "retinal metabolic process"
}